{
  "gene_name": "HORMA domain-containing protein 2",
  "gene_symbol": "HORMAD2",
  "term_label": "synaptonemal complex",
  "term_id": "GO:0000795",
  "gene": "UniProtKB:Q8N7B1"
}